{
  "gene": "UniProtKB:Q8NH60",
  "term_id": "GO:0005886",
  "gene_symbol": "OR52J3",
  "gene_name": "Olfactory receptor 52J3",
  "term_label": "plasma membrane"
}